{
  "term_label": "extracellular space",
  "gene_name": "Cystatin-SN",
  "term_id": "GO:0005615",
  "gene_symbol": "CST1",
  "gene": "UniProtKB:P01037"
}